{
  "term_id": "GO:0047837",
  "term_label": "D-xylose 1-dehydrogenase (NADP+) activity",
  "gene_name": "Trans-1,2-dihydrobenzene-1,2-diol dehydrogenase",
  "gene_symbol": "DHDH",
  "gene": "UniProtKB:Q9UQ10"
}